{
  "gene_symbol": "MX1",
  "gene_name": "Interferon-induced GTP-binding protein Mx1",
  "gene": "UniProtKB:P20591",
  "term_label": "plasma membrane",
  "term_id": "GO:0005886"
}